{
  "gene_name": "Interleukin-6 receptor subunit beta",
  "gene_symbol": "IL6ST",
  "term_label": "positive regulation of cell population proliferation",
  "gene": "UniProtKB:P40189",
  "term_id": "GO:0008284"
}